{
  "term_label": "semaphorin receptor binding",
  "gene_symbol": "SEMA6A",
  "gene_name": "Semaphorin-6A",
  "gene": "UniProtKB:Q9H2E6",
  "term_id": "GO:0030215"
}